{
  "gene": "UniProtKB:Q9Y2W1",
  "term_label": "positive regulation of transcription by RNA polymerase II",
  "gene_symbol": "THRAP3",
  "term_id": "GO:0045944",
  "gene_name": "Thyroid hormone receptor-associated protein 3"
}